retinal rod cell differentiation [GO:0060221] (biological process) Sources: GOC:dph Relationships: is a type of camera-type eye photoreceptor cell differentiation [GO:0060219] Definition: The process in which a relatively unspecialized cell acquires the specialized features of a retinal rod cell.